lipoate catabolic process [GO:0032323] (biological process) Also known as: lipoic acid breakdown, lipoic acid catabolism, lipoic acid degradation Relationships: is a type of GO:0009062; is a type of lipoate metabolic process [GO:0009106]; is a type of sulfur compound catabolic process [GO:0044273] Sources: GOC:mah Definition: The chemical reactions and pathways resulting in the breakdown of lipoate.